{
  "gene_name": "C-terminal-binding protein 2",
  "gene": "UniProtKB:P56545",
  "term_label": "regulation of transcription by RNA polymerase II",
  "term_id": "GO:0006357",
  "gene_symbol": "CTBP2"
}